{
  "gene_symbol": "FAM86C2P",
  "term_id": "UNKNOWN:0003",
  "gene": "UniProtKB:A6NEL3",
  "term_label": "Unknown cellular component",
  "gene_name": "Putative protein FAM86C2P"
}